histamine secretion by basophil [GO:0002557] (biological process) Sources: GOC:add, ISBN:0781735149 Relationships: is a type of histamine secretion involved in inflammatory response [GO:0002441]; is a type of establishment of localization in cell [GO:0051649]; is a type of exocytic process [GO:0140029]; is part of basophil degranulation [GO:0002561] Definition: The regulated release of histamine by a basophil or group of basophils.